{
  "gene": "UniProtKB:Q9BV73",
  "term_label": "centrosome",
  "term_id": "GO:0005813",
  "gene_symbol": "CEP250",
  "gene_name": "Centrosome-associated protein CEP250"
}